regulation of xenobiotic detoxification by transmembrane export across the plasma membrane [GO:1905699] (biological process) Relationships: is_a regulation of transmembrane transport [GO:0034762]; is a type of regulation of response to drug [GO:2001023]; regulates xenobiotic detoxification by transmembrane export across the plasma membrane [GO:1990961] References: PMID:15198509 Sources: GOC:TermGenie, GOC:krc, GO_REF:0000058 Also known as: regulation of drug transmembrane export, regulation of xenobiotic transmembrane export Subtypes: negative regulation of xenobiotic detoxification by transmembrane export across the plasma membrane [GO:1905700], GO:1905701 Definition: Any process that modulates the frequency, rate or extent of xenobiotic transmembrane export. A xenobiotic is a compound foreign to the organism exposed to it. It may be synthesized by another organism (like ampicilin) or it can be a synthetic chemical.